{
  "term_label": "cytoplasm",
  "gene": "UniProtKB:Q9H568",
  "term_id": "GO:0005737",
  "gene_symbol": "ACTL8",
  "gene_name": "Actin-like protein 8"
}